{
  "gene": "UniProtKB:Q9NYC9",
  "term_label": "dynein complex",
  "term_id": "GO:0030286",
  "gene_name": "Dynein axonemal heavy chain 9",
  "gene_symbol": "DNAH9"
}